{
  "gene_symbol": "TOR1AIP2",
  "term_id": "GO:0007029",
  "term_label": "endoplasmic reticulum organization",
  "gene": "UniProtKB:Q8NFQ8",
  "gene_name": "Torsin-1A-interacting protein 2"
}